maintenance of postsynaptic density structure [GO:0099562] (biological process) Definition: A process which maintains the organization and the arrangement of proteins in the presynaptic density. Sources: GOC:dos Relationships: is a type of maintenance of postsynaptic specialization structure [GO:0098880]